N-acylsphingosine amidohydrolase activity [GO:0017040] (molecular function) Also known as: glycosphingolipid ceramide deacylase, ceramidase activity, acylsphingosine deacylase activity Definition: Catalysis of the reaction: an N-acylsphing-4-enine + H2O = a fatty acid + sphing-4-enine. Relationships: is_a GO:0016811 Sources: RHEA:20856